{
  "gene": "UniProtKB:O00445",
  "term_label": "regulation of calcium ion-dependent exocytosis",
  "gene_symbol": "SYT5",
  "gene_name": "Synaptotagmin-5",
  "term_id": "GO:0017158"
}